{
  "gene": "UniProtKB:Q13424",
  "term_id": "GO:0017080",
  "gene_name": "Alpha-1-syntrophin",
  "gene_symbol": "SNTA1",
  "term_label": "sodium channel regulator activity"
}